{
  "term_label": "Unknown molecular function",
  "gene_name": "Ankyrin repeat domain-containing protein 53",
  "gene": "UniProtKB:Q8N9V6",
  "gene_symbol": "ANKRD53",
  "term_id": "UNKNOWN:0001"
}